{
  "term_label": "RNA polymerase II general transcription initiation factor activity",
  "term_id": "GO:0016251",
  "gene_name": "TATA-box-binding protein-associated factor 11-like protein 5",
  "gene_symbol": "TAF11L5",
  "gene": "UniProtKB:A0A1W2PP81"
}